{
  "term_label": "DNA-binding transcription factor activity, RNA polymerase II-specific",
  "gene_symbol": "RFX8",
  "gene_name": "DNA-binding protein RFX8",
  "gene": "UniProtKB:Q6ZV50",
  "term_id": "GO:0000981"
}